{
  "term_id": "UNKNOWN:0002",
  "term_label": "Unknown biological process",
  "gene_symbol": "LY6L",
  "gene": "UniProtKB:H3BQJ8",
  "gene_name": "Lymphocyte antigen 6L"
}